{
  "gene": "UniProtKB:Q86TB9",
  "term_label": "deadenylation-dependent decapping of nuclear-transcribed mRNA",
  "gene_symbol": "PATL1",
  "term_id": "GO:0000290",
  "gene_name": "Protein PAT1 homolog 1"
}